{
  "gene_symbol": "C11orf16",
  "gene_name": "Uncharacterized protein C11orf16",
  "term_id": "UNKNOWN:0002",
  "gene": "UniProtKB:Q9NQ32",
  "term_label": "Unknown biological process"
}